ESCRT complex assembly [GO:1904895] (biological process) References: PMID:21118109 Sources: GOC:PARL, GOC:TermGenie, GOC:pad, GO_REF:0000079 Subtypes: ESCRT III complex assembly [GO:1904902] Also known as: ESCRT complex formation, endosomal sorting complex required for transport assembly, endosomal sorting complex required for transport formation Definition: The aggregation, arrangement and bonding together of a set of components to form an ESCRT complex. Relationships: is a type of protein-containing complex assembly [GO:0065003]